{
  "gene_name": "Protein Wnt-7a",
  "gene_symbol": "WNT7A",
  "gene": "UniProtKB:O00755",
  "term_id": "GO:0005125",
  "term_label": "cytokine activity"
}